{
  "term_label": "thyrotropin-releasing hormone receptor binding",
  "gene_symbol": "GPHA2",
  "gene": "UniProtKB:Q96T91",
  "term_id": "GO:0031531",
  "gene_name": "Glycoprotein hormone alpha-2"
}